{
  "gene_name": "BEN domain-containing protein 3",
  "gene": "UniProtKB:Q5T5X7",
  "term_id": "GO:0000122",
  "gene_symbol": "BEND3",
  "term_label": "negative regulation of transcription by RNA polymerase II"
}